toxic metabolite repair [GO:0110052] (biological process) Definition: A cellular process that, through single- or multi-step enzymatic reactions, repairs toxic endogenous compounds, formed as by-products of primary metabolism, by converting them into useful metabolites. References: PMID:23334546 Sources: GOC:ka, GOC:vw Relationships: is a type of metabolite repair [GO:0110051]; is a type of GO:1990748